type 1F serotonin receptor binding [GO:0031825] (molecular function) Also known as: 5-hydroxytryptamine 1F receptor binding, type 1F serotonin receptor ligand Sources: GOC:mah, GOC:nln Definition: Binding to a type 1F serotonin receptor. Relationships: is a type of G protein-coupled serotonin receptor binding [GO:0031821]